indoleacetic acid amide conjugate biosynthetic process [GO:0033475] (biological process) Also known as: IAA amide conjugate biosynthetic process, indole acetic acid amide conjugate biosynthesis, indole acetic acid amide conjugate biosynthetic process, indoleacetic acid amide conjugate anabolism, indoleacetic acid amide conjugate biosynthesis, indoleacetic acid amide conjugate formation, indoleacetic acid amide conjugate synthesis Relationships: is a type of indoleacetic acid conjugate biosynthetic process [GO:0033474]; is a type of GO:0043604 Sources: GOC:mah, MetaCyc:PWY-1782 Definition: The chemical reactions and pathways resulting in the formation of an indole-3-acetic acid amide conjugate, a form of indoleacetic acid covalently bound to an amino acid or polypeptide through an amide bond.